{
  "gene_symbol": "NOX4",
  "gene": "UniProtKB:Q9NPH5",
  "gene_name": "NADPH oxidase 4",
  "term_id": "GO:0042554",
  "term_label": "superoxide anion generation"
}